{
  "gene_name": "Transcription factor HES-4",
  "term_label": "negative regulation of transcription by RNA polymerase II",
  "term_id": "GO:0000122",
  "gene": "UniProtKB:Q9HCC6",
  "gene_symbol": "HES4"
}